retrograde transport, endosome to Golgi [GO:0042147] (BP) Relationships: is_a endosomal transport [GO:0016197]; is a type of cytosolic transport [GO:0016482] Definition: The directed movement of membrane-bounded vesicles from endosomes back to the trans-Golgi network where they are recycled for further rounds of transport. Subtypes: early endosome to Golgi transport [GO:0034498], late endosome to Golgi transport [GO:0034499], recycling endosome to Golgi transport [GO:0071955] Also known as: retrograde (endosome to Golgi) transport References: PMID:10873832, PMID:16936697 Sources: GOC:jl Regulation: regulated by regulation of retrograde transport, endosome to Golgi [GO:1905279]; negatively regulated by GO:1905280; RO_0002213 by GO:1905281